{
  "gene_symbol": "PSMA7",
  "term_id": "UNKNOWN:0001",
  "gene": "UniProtKB:O14818",
  "term_label": "Unknown molecular function",
  "gene_name": "Proteasome subunit alpha type-7"
}